{
  "gene": "UniProtKB:Q13901",
  "gene_symbol": "C1D",
  "term_label": "RNA binding",
  "gene_name": "Nuclear nucleic acid-binding protein C1D",
  "term_id": "GO:0003723"
}